{
  "gene_symbol": "CBLN2",
  "term_label": "Unknown molecular function",
  "gene": "UniProtKB:Q8IUK8",
  "term_id": "UNKNOWN:0001",
  "gene_name": "Cerebellin-2"
}